{
  "term_id": "GO:0008191",
  "gene_symbol": "BST2",
  "gene_name": "Bone marrow stromal antigen 2",
  "term_label": "metalloendopeptidase inhibitor activity",
  "gene": "UniProtKB:Q10589"
}